{
  "gene": "UniProtKB:Q96AQ9",
  "term_id": "UNKNOWN:0001",
  "gene_name": "Protein FAM131C",
  "gene_symbol": "FAM131C",
  "term_label": "Unknown molecular function"
}